{
  "gene": "UniProtKB:Q9H8P0",
  "term_label": "dolichyl monophosphate biosynthetic process",
  "term_id": "GO:0043048",
  "gene_symbol": "SRD5A3",
  "gene_name": "Polyprenol reductase"
}